positive regulation of oocyte karyosome formation [GO:0120315] (biological process) References: PMID:33382409 Sources: GOC:ha, GOC:krc Relationships: is_a positive regulation of cell cycle process [GO:0090068]; is a type of regulation of oocyte karyosome formation [GO:0120313]; is a type of positive regulation of reproductive process [GO:2000243]; is a type of positive regulation of chromosome organization [GO:2001252]; positively regulates oocyte karyosome formation [GO:0030717] Definition: Any process that activates or increases the frequency, rate or extent of oocyte karyosome formation, the chromosome organization process in which meiotic chromosomes in the oocyte nucleus cluster together to form a compact spherical structure called the karyosome.